phosphatidylcholine biosynthesis from phosphoryl-ethanolamine via N-dimethylethanolamine phosphate and CDP-N-dimethylethanolamine [GO:0070834] (BP) Definition: The phosphatidylcholine biosynthetic process that begins with two N-methylations with phospho-base phosphoethanolamine and phospho-N-methylethanolamine, followed by a downstream N-methylation on phosphatidyl-base phosphatidyl-N-dimethylethanolamine; the process ends with the conversion of a phosphatidyl-N-dimethylethanolamine to a phosphatidylcholine. Relationships: is a type of phosphatidylcholine biosynthetic process [GO:0006656] Sources: MetaCyc:PWY4FS-4